carotenoid transport [GO:0046867] (BP) Sources: GOC:ai Relationships: is_a tetraterpenoid transport [GO:0046866] Definition: The directed movement of carotenoids into, out of or within a cell, or between cells, by means of some agent such as a transporter or pore. Carotenoids are tetraterpenoid compounds in which two units of 4 isoprenoid residues joined head-to-tail are themselves joined tail-to-tail.